root morphogenesis [GO:0010015] (biological process) Subtypes: embryonic root morphogenesis [GO:0010086], post-embryonic root morphogenesis [GO:0010101] Definition: The process in which the anatomical structures of roots are generated and organized. The root is the usually underground part of a seed plant body that originates from the hypocotyl, functions as an organ of absorption, aeration, and food storage or as a means of anchorage and support. Relationships: is a type of plant organ morphogenesis [GO:1905392]; is part of root development [GO:0048364] Sources: GOC:sm, ISBN:0877797099 Regulation: regulated by regulation of root morphogenesis [GO:2000067]